{
  "term_label": "Unknown molecular function",
  "term_id": "UNKNOWN:0001",
  "gene": "UniProtKB:Q8WUJ1",
  "gene_symbol": "CYB5D2",
  "gene_name": "Neuferricin"
}